{
  "gene_symbol": "PBK",
  "gene": "UniProtKB:Q96KB5",
  "gene_name": "Lymphokine-activated killer T-cell-originated protein kinase",
  "term_label": "Unknown cellular component",
  "term_id": "UNKNOWN:0003"
}